protein-glutamine gamma-glutamyltransferase activity [GO:0003810] (MF) Definition: Catalysis of the reaction: L-glutaminyl-[protein] + L-lysyl-[protein] = [protein]-L-lysyl-N(6)-5-L-glutamyl-[protein] + NH4+. This reaction is the formation of the N6-(L-isoglutamyl)-L-lysine isopeptide, resulting in cross-linking polypeptide chains; the gamma-carboxamide groups of peptidyl-glutamine residues act as acyl donors, and the 6-amino-groups of peptidyl-lysine residues act as acceptors, to give intra- and intermolecular N6-(5-glutamyl)lysine cross-links. Sources: EC:2.3.2.13 Relationships: is a type of aminoacyltransferase activity [GO:0016755]; is a type of catalytic activity, acting on a protein [GO:0140096] Also known as: TGase activity, fibrinoligase activity, transglutaminase activity, tissue transglutaminase, R-glutaminyl-peptide:amine gamma-glutamyl transferase activity, factor XIIIa, fibrin stabilizing factor, glutaminylpeptide gamma-glutamyltransferase activity, polyamine transglutaminase activity, protein-glutamine:amine gamma-glutamyltransferase Regulation: positively regulated by positive regulation of protein-glutamine gamma-glutamyltransferase activity [GO:0150074]